{
  "gene_symbol": "STAT5A",
  "term_label": "nucleus",
  "gene_name": "Signal transducer and activator of transcription 5A",
  "gene": "UniProtKB:P42229",
  "term_id": "GO:0005634"
}